{
  "term_label": "cilium",
  "gene_symbol": "ANKS3",
  "gene": "UniProtKB:Q6ZW76",
  "term_id": "GO:0005929",
  "gene_name": "Ankyrin repeat and SAM domain-containing protein 3"
}